testosterone 16-alpha-hydroxylase activity [GO:0008390] (molecular function) Relationships: is a type of steroid hydroxylase activity [GO:0008395]; is_a oxidoreductase activity, acting on paired donors, with incorporation or reduction of molecular oxygen, reduced flavin or flavoprotein as one donor, and incorporation of one atom of oxygen [GO:0016712] Sources: RHEA:53196 Also known as: cytochrome P450 CYP2B10, cytochrome P450 CYP2B9, cytochrome P450 CYP2D10, cytochrome P450 CYP2D11, cytochrome P450 CYP2D9 Definition: Catalysis of the reaction: O2 + reduced [NADPH--hemoprotein reductase] + testosterone = 16alpha,17beta-dihydroxyandrost-4-en-3-one + H+ + H2O + oxidized [NADPH--hemoprotein reductase].